{
  "term_label": "cis-Golgi network",
  "gene_name": "Golgin subfamily A member 8B",
  "gene_symbol": "GOLGA8B",
  "term_id": "GO:0005801",
  "gene": "UniProtKB:A8MQT2"
}